{
  "gene": "UniProtKB:Q8IZP0",
  "term_id": "GO:0001764",
  "gene_name": "Abl interactor 1",
  "gene_symbol": "ABI1",
  "term_label": "neuron migration"
}